{
  "gene_symbol": "HEATR4",
  "gene": "UniProtKB:Q86WZ0",
  "term_label": "Unknown biological process",
  "gene_name": "HEAT repeat-containing protein 4",
  "term_id": "UNKNOWN:0002"
}